{
  "gene_symbol": "TMEM89",
  "term_id": "UNKNOWN:0001",
  "term_label": "Unknown molecular function",
  "gene_name": "Transmembrane protein 89",
  "gene": "UniProtKB:A2RUT3"
}